{
  "gene_symbol": "HCRT",
  "term_label": "perinuclear region of cytoplasm",
  "gene_name": "Hypocretin neuropeptide precursor",
  "gene": "UniProtKB:O43612",
  "term_id": "GO:0048471"
}